{
  "gene_name": "26S proteasome non-ATPase regulatory subunit 9",
  "term_id": "UNKNOWN:0001",
  "term_label": "Unknown molecular function",
  "gene_symbol": "PSMD9",
  "gene": "UniProtKB:O00233"
}